oxygen metabolic process [GO:0072592] (biological process) Also known as: diatomic oxygen metabolic process, oxygen metabolism Relationships: is a type of metabolic process [GO:0008152] Sources: GOC:mah Definition: The chemical reactions and pathways involving diatomic oxygen (O2). Regulation: regulated by regulation of oxygen metabolic process [GO:2000374]